{
  "gene_name": "E3 ubiquitin-protein ligase CCNB1IP1",
  "gene_symbol": "CCNB1IP1",
  "term_id": "GO:0007131",
  "gene": "UniProtKB:Q9NPC3",
  "term_label": "reciprocal meiotic recombination"
}